vegetative meristem growth [GO:0010448] (biological process) Definition: The increase in size or mass of a vegetative meristem, a population of undifferentiated cells in a plant shoot which maintains a continuous balance between the production of stem cells and the incorporation of their derivatives into lateral organ primordia. Sources: GOC:tb, ISBN:0849397928 Relationships: is a type of meristem growth [GO:0035266]; is a type of developmental vegetative growth [GO:0080186]; is part of shoot system development [GO:0048367] Regulation: regulated by regulation of vegetative meristem growth [GO:0010083]